{
  "term_label": "Unknown biological process",
  "gene": "UniProtKB:A0A0A0MT82",
  "gene_name": "Immunoglobulin lambda joining 2 (Fragment)",
  "term_id": "UNKNOWN:0002",
  "gene_symbol": "IGLJ2"
}